{
  "gene": "UniProtKB:P61236",
  "gene_name": "Protein yippee-like 3",
  "gene_symbol": "YPEL3",
  "term_id": "UNKNOWN:0001",
  "term_label": "Unknown molecular function"
}